{
  "term_id": "GO:0004864",
  "gene_name": "Alpha-endosulfine",
  "gene": "UniProtKB:O43768",
  "gene_symbol": "ENSA",
  "term_label": "protein phosphatase inhibitor activity"
}